regulation of cytochrome-c oxidase activity [GO:1904959] (biological process) Subtypes: positive regulation of cytochrome-c oxidase activity [GO:1904960] References: PMID:26734017 Sources: GOC:TermGenie, GO_REF:0000059 Also known as: regulation of NADH cytochrome c oxidase, regulation of cytochrome c oxidase activity, regulation of aa3-type cytochrome c oxidase, regulation of ba3-type cytochrome c oxidase, regulation of caa3-type cytochrome c oxidase, regulation of cbb3-type cytochrome c oxidase, regulation of cytochrome a3 activity, regulation of cytochrome aa3 activity, regulation of ferrocytochrome c oxidase, regulation of ferrocytochrome-c:oxygen oxidoreductase, regulation of indophenol oxidase, regulation of indophenolase, regulation of complex IV (mitochondrial electron transport) activity, regulation of cytochrome oxidase activity, regulation of warburg's respiratory enzyme activity Relationships: is a type of GO:0010155; is a type of regulation of transmembrane transporter activity [GO:0022898]; regulates GO:0004129 Definition: Any process that modulates the frequency, rate or extent of cytochrome-c oxidase activity.